{
  "gene": "UniProtKB:P55211",
  "term_label": "cytoplasm",
  "gene_symbol": "CASP9",
  "gene_name": "Caspase-9",
  "term_id": "GO:0005737"
}